{
  "gene_symbol": "ACLY",
  "gene": "UniProtKB:P53396",
  "gene_name": "ATP-citrate synthase",
  "term_id": "GO:0006085",
  "term_label": "acetyl-CoA biosynthetic process"
}